{
  "term_label": "protein kinase binding",
  "gene_symbol": "FAM83F",
  "gene": "UniProtKB:Q8NEG4",
  "gene_name": "Protein FAM83F",
  "term_id": "GO:0019901"
}